{
  "gene": "UniProtKB:A0A1W2PR95",
  "gene_name": "Immunoglobulin-binding protein 1 family member C",
  "gene_symbol": "IGBP1C",
  "term_label": "protein phosphatase 2A binding",
  "term_id": "GO:0051721"
}